{
  "gene": "UniProtKB:Q9NX70",
  "gene_name": "Mediator of RNA polymerase II transcription subunit 29",
  "term_id": "GO:0003712",
  "gene_symbol": "MED29",
  "term_label": "transcription coregulator activity"
}